C bouton [GO:1990024] (cellular component) Definition: Synaptic bouton found in spinal cord on the soma and proximal dendrites of motor neurons. Sources: NIF_Subcellular:nlx_subcell_100208 Relationships: is_a GO:0043195